histone H1R54 arginine deiminase activity [GO:0140810] (molecular function) Definition: Catalysis of the reaction: H2O + histone H1 L-arginyl (position 54)= histone H1 L-citrullyl (position 54) + NH4+, resulting in histone H1 citrullination at position 54. References: PMID:24463520 Note: The substrate for histone deiminase may be methyl-arginine, rather than arginine (see PMID:35197210 and PMID:16567635). Also known as: H1-R54 citrullination, histone H1-R54 deiminase activity, histone-arginine deiminase activity (H1-R54 specific) Relationships: is_a histone arginine deiminase activity [GO:0140794]